{
  "term_id": "GO:0007155",
  "gene_name": "Protocadherin gamma-C4",
  "term_label": "cell adhesion",
  "gene": "UniProtKB:Q9Y5F7",
  "gene_symbol": "PCDHGC4"
}